{
  "term_label": "DNA-binding transcription factor activity, RNA polymerase II-specific",
  "gene_symbol": "TP53",
  "term_id": "GO:0000981",
  "gene": "UniProtKB:P04637",
  "gene_name": "Cellular tumor antigen p53"
}